{
  "gene": "UniProtKB:Q9BW04",
  "term_id": "UNKNOWN:0001",
  "term_label": "Unknown molecular function",
  "gene_symbol": "SARG",
  "gene_name": "Specifically androgen-regulated gene protein"
}